{
  "term_label": "positive regulation of JNK cascade",
  "gene_symbol": "NRK",
  "term_id": "GO:0046330",
  "gene_name": "Nik-related protein kinase",
  "gene": "UniProtKB:Q7Z2Y5"
}